{
  "gene": "UniProtKB:P46108",
  "gene_symbol": "CRK",
  "term_label": "enzyme-linked receptor protein signaling pathway",
  "gene_name": "Adapter molecule crk",
  "term_id": "GO:0007167"
}